{
  "gene_symbol": "C19orf44",
  "term_id": "UNKNOWN:0001",
  "gene": "UniProtKB:Q9H6X5",
  "term_label": "Unknown molecular function",
  "gene_name": "Uncharacterized protein C19orf44"
}